{
  "gene": "UniProtKB:Q99805",
  "gene_symbol": "TM9SF2",
  "term_id": "GO:0072657",
  "term_label": "protein localization to membrane",
  "gene_name": "Transmembrane 9 superfamily member 2"
}